response to silver ion [GO:0010272] (biological process) Subtypes: cellular response to silver ion [GO:0071292] Relationships: is a type of response to metal ion [GO:0010038] Definition: Any process that results in a change in state or activity of a cell or an organism (in terms of movement, secretion, enzyme production, gene expression, etc.) as a result of a silver ion stimulus. References: PMID:16367966